symbiont cell surface [GO:0106139] (CC) References: PMID:30049880 Sources: GOC:rjd Definition: The cell surface of a secondary, endosymbiont organism with which the first organism is interacting. The symbiont is defined as the smaller of the organisms involved in a symbiotic interaction. Relationships: is a type of other organism part [GO:0044217] Also known as: endosymbiont cell surface